{
  "term_label": "Arp2/3 complex-mediated actin nucleation",
  "term_id": "GO:0034314",
  "gene_symbol": "JMY",
  "gene": "UniProtKB:Q8N9B5",
  "gene_name": "Junction-mediating and -regulatory protein"
}